tumor necrosis factor production [GO:0032640] (biological process) References: PMID:10891884, PMID:15560120 Sources: GOC:mah Relationships: is a type of GO:0071706 Also known as: TNF production, cachectin production, TNF alpha biosynthesis, TNF biosynthesis, TNF biosynthetic process, TNF-alpha biosynthesis, TNF-alpha biosynthetic process, tumor necrosis factor anabolism, tumor necrosis factor biosynthesis, tumor necrosis factor biosynthetic process, tumor necrosis factor formation, tumor necrosis factor secretion, tumor necrosis factor synthesis, TNF-alpha production, Tnfa production, tumor necrosis factor-alpha production Definition: The appearance of tumor necrosis factor due to biosynthesis or secretion following a cellular stimulus, resulting in an increase in its intracellular or extracellular levels. Tumor necrosis factor is an inflammatory cytokine produced by macrophages/monocytes during acute inflammation and which is responsible for a diverse range of signaling events within cells, leading to necrosis or apoptosis. Regulation: regulated by regulation of tumor necrosis factor production [GO:0032680]; negatively regulated by negative regulation of tumor necrosis factor production [GO:0032720]; positively regulated by positive regulation of tumor necrosis factor production [GO:0032760] Note: Note that this term refers only to the specific, original 'tumor necrosis factor' protein (TNF) and not other members of the tumor necrosis factor superfamily (those with the gene symbol root 'TNFSF'). That this term is in the subset of terms that should not be used for direct gene product annotation. Instead, select one of the 'regulation' children terms.